{
  "term_id": "GO:0005200",
  "gene_name": "Actin, alpha cardiac muscle 1",
  "gene": "UniProtKB:P68032",
  "term_label": "structural constituent of cytoskeleton",
  "gene_symbol": "ACTC1"
}